{
  "term_id": "UNKNOWN:0002",
  "gene_symbol": "SAP25",
  "gene": "UniProtKB:Q8TEE9",
  "gene_name": "Histone deacetylase complex subunit SAP25",
  "term_label": "Unknown biological process"
}